{
  "term_label": "catenin complex",
  "gene": "UniProtKB:P55289",
  "term_id": "GO:0016342",
  "gene_name": "Cadherin-12",
  "gene_symbol": "CDH12"
}